{
  "gene_symbol": "TPPP",
  "gene_name": "Tubulin polymerization-promoting protein",
  "term_label": "tubulin binding",
  "gene": "UniProtKB:O94811",
  "term_id": "GO:0015631"
}